thiamine-phosphate diphosphorylase activity [GO:0004789] (molecular function) Definition: Catalysis of the reaction: 4-amino-2-methyl-5-diphosphomethylpyrimidine + 4-methyl-5-(2-phosphoethyl)-thiazole + H+ = diphosphate + thiamine phosphate. Sources: EC:2.5.1.3, RHEA:22328 Also known as: thiamin-phosphate diphosphorylase activity, thiamin-phosphate pyrophosphorylase activity, thiamine-phosphate pyrophosphorylase activity, 2-methyl-4-amino-5-hydroxymethylpyrimidine-diphosphate:4-methyl-5-(2-phosphoethyl)thiazole 2-methyl-4-aminopyrimidine-5-methenyltransferase activity, TMP diphosphorylase activity, TMP pyrophosphorylase activity, TMP-PPase activity, thiamine monophosphate pyrophosphorylase activity, thiamine phosphate pyrophosphorylase activity, thiamine-phosphate synthase activity Relationships: is a type of transferase activity, transferring alkyl or aryl (other than methyl) groups [GO:0016765]